{
  "term_id": "UNKNOWN:0001",
  "gene": "UniProtKB:Q9BV73",
  "gene_name": "Centrosome-associated protein CEP250",
  "gene_symbol": "CEP250",
  "term_label": "Unknown molecular function"
}